{
  "term_label": "Unknown biological process",
  "gene_symbol": "MCF2L2",
  "term_id": "UNKNOWN:0002",
  "gene": "UniProtKB:Q86YR7",
  "gene_name": "Probable guanine nucleotide exchange factor MCF2L2"
}